peripheral nervous system neuron axonogenesis [GO:0048936] (biological process) Definition: Generation of a long process from a neuron whose cell body resides in the peripheral nervous system. The axon carries action potential from the cell body towards target cells. Relationships: is a type of axonogenesis [GO:0007409]; is part of GO:0048935 Sources: GOC:dgh